flavonoid sulfotransferase activity [GO:1990135] (molecular function) References: PMID:23611783 Definition: Catalysis of the reaction: a flavonoid + 3'-phosphoadenosine-5'-phosphosulfate = sulfated flavonoid + adenosine-3',5'-diphosphate. This reaction is the transfer of a sulfate group to the hydroxyl group of a flavonoid acceptor, producing the sulfated flavonoid derivative. Relationships: is_a sulfotransferase activity [GO:0008146]